{
  "term_label": "regulation of inflammatory response",
  "gene_symbol": "CASP1",
  "gene_name": "Caspase-1",
  "term_id": "GO:0050727",
  "gene": "UniProtKB:P29466"
}